{
  "gene": "UniProtKB:A0A075B6X4",
  "term_label": "Unknown molecular function",
  "term_id": "UNKNOWN:0001",
  "gene_symbol": "TRAJ28",
  "gene_name": "T cell receptor alpha joining 28 (Fragment)"
}